mesenchymal to epithelial transition involved in renal vesicle formation [GO:0072036] (biological process) Definition: A transition where a mesenchymal cell establishes apical/basolateral polarity,forms intercellular adhesive junctions, synthesizes basement membrane components and becomes an epithelial cell that will contribute to the shaping of the renal vesicle. Relationships: is a type of GO:0035850; is a type of mesenchymal to epithelial transition [GO:0060231]; is part of renal vesicle formation [GO:0072033] Subtypes: mesenchymal to epithelial transition involved in mesonephric renal vesicle formation [GO:0061271], mesenchymal to epithelial transition involved in metanephric renal vesicle formation [GO:0072285] Sources: GOC:mtg_kidney_jan10